{
  "term_id": "GO:1990825",
  "gene_symbol": "ETF1",
  "gene_name": "Eukaryotic peptide chain release factor subunit 1",
  "term_label": "sequence-specific mRNA binding",
  "gene": "UniProtKB:P62495"
}